{
  "gene": "UniProtKB:O94812",
  "gene_symbol": "BAIAP3",
  "gene_name": "BAI1-associated protein 3",
  "term_label": "SNARE binding",
  "term_id": "GO:0000149"
}